{
  "gene_symbol": "IL17F",
  "gene": "UniProtKB:Q96PD4",
  "term_id": "GO:0005125",
  "gene_name": "Interleukin-17F",
  "term_label": "cytokine activity"
}